SMC loading complex [GO:0032116] (cellular component) Definition: A protein complex required for the loading of a structural maintenance of chromosome (SMC) complex, such as cohesin, condensin or SMC5/SMC6, onto DNA. Appears to be eukaryotically conserved. References: PMID:10882066 Sources: GOC:curators, GOC:vw Also known as: SCC2/SCC4 loading complex, cohesin loading complex, chromatin loading complex Relationships: is a type of GO:0140513 Subtypes: Scc2-Scc4 cohesin loading complex [GO:0090694], Wpl/Pds5 cohesin loading/unloading complex [GO:0090695]